{
  "gene": "UniProtKB:Q9Y342",
  "term_id": "GO:0016020",
  "gene_name": "Plasmolipin",
  "term_label": "membrane",
  "gene_symbol": "PLLP"
}